{
  "gene_name": "Inward rectifier potassium channel 2",
  "gene": "UniProtKB:P63252",
  "gene_symbol": "KCNJ2",
  "term_id": "GO:1990573",
  "term_label": "potassium ion import across plasma membrane"
}